{
  "gene": "UniProtKB:Q9H981",
  "gene_symbol": "ACTR8",
  "term_label": "mRNA binding",
  "term_id": "GO:0003729",
  "gene_name": "Actin-related protein 8"
}